{
  "gene_symbol": "STAC",
  "gene": "UniProtKB:Q99469",
  "gene_name": "SH3 and cysteine-rich domain-containing protein",
  "term_label": "transmembrane transporter binding",
  "term_id": "GO:0044325"
}